{
  "gene_symbol": "PPP1R13L",
  "gene": "UniProtKB:Q8WUF5",
  "gene_name": "RelA-associated inhibitor",
  "term_id": "GO:0045597",
  "term_label": "positive regulation of cell differentiation"
}